squalene-hopene cyclase activity [GO:0051007] (molecular function) Relationships: is_a intramolecular transferase activity [GO:0016866]; is a type of squalene cyclase activity [GO:0034072] Also known as: squalene:hopene cyclase activity, squalene mutase (cyclizing) Sources: EC:5.4.99.17 Definition: Catalysis of the reaction: squalene = hop-22(29)-ene.